{
  "gene_name": "Sodium channel subunit beta-3",
  "term_id": "GO:0035725",
  "gene_symbol": "SCN3B",
  "gene": "UniProtKB:Q9NY72",
  "term_label": "sodium ion transmembrane transport"
}